{
  "gene": "UniProtKB:Q3ZCX4",
  "term_id": "GO:0005634",
  "gene_symbol": "ZNF568",
  "gene_name": "Zinc finger protein 568",
  "term_label": "nucleus"
}